{
  "term_id": "UNKNOWN:0002",
  "gene_symbol": "LINC00242",
  "gene": "UniProtKB:Q5T6M2",
  "term_label": "Unknown biological process",
  "gene_name": "Putative uncharacterized protein encoded by LINC00242"
}